enzyme-substrate adaptor activity [GO:0140767] (molecular function) Definition: An adaptor that brings together an enzyme and its substrate. Adaptors recruit the substrate to its enzyme, thus contributing to substrate selection and specificity. References: PMID:16250895, PMID:34358446 Also known as: protein-substrate adaptor activity, protein substrate chaperone activity Relationships: is a type of protein-macromolecule adaptor activity [GO:0030674] Subtypes: protein ADP-ribosyltransferase-substrate adaptor activity [GO:0140768], GO:1990756